{
  "gene": "UniProtKB:Q9NQ48",
  "gene_symbol": "LZTFL1",
  "gene_name": "Leucine zipper transcription factor-like protein 1",
  "term_id": "UNKNOWN:0001",
  "term_label": "Unknown molecular function"
}